regulation of cellobiose catabolic process [GO:1900282] (biological process) Definition: Any process that modulates the frequency, rate or extent of cellobiose catabolic process. Relationships: is a type of regulation of carbohydrate catabolic process [GO:0043470]; regulates cellobiose catabolic process [GO:2000892] Sources: GOC:TermGenie, GOC:mengo_curators Subtypes: negative regulation of cellobiose catabolic process [GO:1900283], positive regulation of cellobiose catabolic process [GO:1900284] Also known as: regulation of cellobiose catabolism